{
  "term_label": "Golgi to vacuole transport",
  "gene_name": "Vacuolar protein sorting-associated protein 52 homolog",
  "gene_symbol": "VPS52",
  "term_id": "GO:0006896",
  "gene": "UniProtKB:Q8N1B4"
}